{
  "gene_symbol": "BOLL",
  "gene": "UniProtKB:Q8N9W6",
  "term_id": "GO:0003730",
  "term_label": "mRNA 3'-UTR binding",
  "gene_name": "Protein boule-like"
}